3',3'-cyclic GMP-AMP synthase activity [GO:0140701] (molecular function) Definition: Catalysis of the reaction: ATP + GTP = 2 diphosphate + cyclic G-P(3'-5')A-P(3'-5') (cyclic 3',3' GAMP). References: PMID:30787435 Sources: RHEA:35647 Also known as: 3',3' cyclic-GAMP synthase activity, 3',3' cyclic-GMP-AMP synthase activity, 3',3'-cyclic GAMP synthase activity Relationships: is a type of GO:0140699